{
  "term_id": "GO:0006886",
  "term_label": "intracellular protein transport",
  "gene_name": "Ras-related protein Rab-32",
  "gene_symbol": "RAB32",
  "gene": "UniProtKB:Q13637"
}